G-protein beta/gamma-subunit complex [GO:0031680] (cellular component) Note: See also the cellular component term 'heterotrimeric G-protein complex ; GO:0005834'. Sources: GOC:mah Also known as: G-beta/G-gamma complex, heterotrimeric G-protein GTPase, beta-subunit Relationships: is a type of GO:0032991; is part of cytoplasm [GO:0005737] Definition: The heterodimer formed by the beta and gamma subunits of a heterotrimeric G protein, which dissociates from the alpha subunit upon guanine nuclotide exchange.